{
  "gene_symbol": "COPZ1",
  "term_label": "intra-Golgi vesicle-mediated transport",
  "term_id": "GO:0006891",
  "gene": "UniProtKB:P61923",
  "gene_name": "Coatomer subunit zeta-1"
}